{
  "gene_name": "Beta-nerve growth factor",
  "term_label": "growth factor activity",
  "gene_symbol": "NGF",
  "term_id": "GO:0008083",
  "gene": "UniProtKB:P01138"
}